{
  "gene_name": "Tumor necrosis factor alpha-induced protein 3",
  "term_id": "GO:0005737",
  "term_label": "cytoplasm",
  "gene": "UniProtKB:P21580",
  "gene_symbol": "TNFAIP3"
}